Cyc8(Ssn6)-Tup1 general repressor complex [GO:0160051] (cellular component) Relationships: is_a RNA polymerase II transcription repressor complex [GO:0090571] Also known as: Tup11/Tup12 repressor complex Definition: A corepressor complex containing the WD-repeat protein Tup1p (S. cerevisiae) and Tup11/Tup12 (fission yeast) and the TPR repeat protein Cyc8p (S. cerevisiae) ssn6 (fission yeast) that is recruited to target genes by DNA-bound repressor proteins preferentially at regions where histones are deacetylated by the Clr6 class I HDAC, and recruits the SWI/SNF and SAGA complexes to promoters. References: PMID:10871883, PMID:17101775, PMID:22156212 Sources: GOC:vw